{
  "term_label": "peptidyl-prolyl cis-trans isomerase activity",
  "gene": "UniProtKB:P62937",
  "term_id": "GO:0003755",
  "gene_name": "Peptidyl-prolyl cis-trans isomerase A",
  "gene_symbol": "PPIA"
}